Golgi cisterna [GO:0031985] (cellular component) Also known as: Golgi apparatus cisterna, Golgi lamellae Definition: Any of the thin, flattened membrane-bounded compartments that form the central portion of the Golgi complex. Relationships: is a type of Golgi apparatus subcompartment [GO:0098791]; is part of Golgi stack [GO:0005795] Sources: GOC:mah Subtypes: GO:0000137, GO:0000138, Golgi medial cisterna [GO:0005797]